{
  "term_label": "chromatin",
  "term_id": "GO:0000785",
  "gene_name": "Akirin-2",
  "gene_symbol": "AKIRIN2",
  "gene": "UniProtKB:Q53H80"
}